{
  "term_label": "calcium/calmodulin-dependent protein kinase activity",
  "gene": "UniProtKB:Q14012",
  "term_id": "GO:0004683",
  "gene_name": "Calcium_calmodulin-dependent protein kinase type 1",
  "gene_symbol": "CAMK1"
}